{
  "term_label": "Unknown cellular component",
  "gene_symbol": "UST",
  "gene": "UniProtKB:Q9Y2C2",
  "gene_name": "Uronyl 2-sulfotransferase",
  "term_id": "UNKNOWN:0003"
}